{
  "gene_symbol": "SMIM17",
  "term_id": "UNKNOWN:0002",
  "gene_name": "Small integral membrane protein 17",
  "gene": "UniProtKB:P0DL12",
  "term_label": "Unknown biological process"
}